{
  "term_id": "UNKNOWN:0001",
  "gene": "UniProtKB:P61565",
  "term_label": "Unknown molecular function",
  "gene_name": "Endogenous retrovirus group K member 21 Env polyprotein",
  "gene_symbol": "ERVK-21"
}